{
  "gene": "UniProtKB:Q02978",
  "gene_symbol": "SLC25A11",
  "term_label": "transmembrane transporter activity",
  "gene_name": "Mitochondrial 2-oxoglutarate_malate carrier protein",
  "term_id": "GO:0022857"
}